{
  "gene_name": "ADP-ribosylation factor 6",
  "term_id": "GO:0016192",
  "gene": "UniProtKB:P62330",
  "term_label": "vesicle-mediated transport",
  "gene_symbol": "ARF6"
}